{
  "term_id": "GO:0006357",
  "gene_symbol": "ZNF174",
  "gene_name": "Zinc finger protein 174",
  "term_label": "regulation of transcription by RNA polymerase II",
  "gene": "UniProtKB:Q15697"
}